{
  "gene_name": "Transmembrane emp24 domain-containing protein 1",
  "gene": "UniProtKB:Q13445",
  "term_id": "UNKNOWN:0001",
  "term_label": "Unknown molecular function",
  "gene_symbol": "TMED1"
}